{
  "gene_symbol": "MYH2",
  "gene_name": "Myosin-2",
  "term_id": "GO:0051015",
  "gene": "UniProtKB:Q9UKX2",
  "term_label": "actin filament binding"
}